{
  "gene": "UniProtKB:O75795",
  "gene_name": "UDP-glucuronosyltransferase 2B17",
  "term_id": "UNKNOWN:0003",
  "term_label": "Unknown cellular component",
  "gene_symbol": "UGT2B17"
}